{
  "gene": "UniProtKB:O43665",
  "gene_name": "Regulator of G-protein signaling 10",
  "term_label": "Unknown biological process",
  "gene_symbol": "RGS10",
  "term_id": "UNKNOWN:0002"
}